{
  "gene": "UniProtKB:Q6PCB0",
  "gene_symbol": "VWA1",
  "term_label": "Unknown biological process",
  "gene_name": "von Willebrand factor A domain-containing protein 1",
  "term_id": "UNKNOWN:0002"
}